regulation of stress fiber assembly [GO:0051492] (biological process) Definition: Any process that modulates the frequency, rate or extent of the assembly of a stress fiber, a bundle of microfilaments and other proteins found in fibroblasts. Relationships: is a type of regulation of actin filament bundle assembly [GO:0032231]; is a type of regulation of actomyosin structure organization [GO:0110020]; regulates stress fiber assembly [GO:0043149] Subtypes: positive regulation of stress fiber assembly [GO:0051496], negative regulation of stress fiber assembly [GO:0051497] Sources: GOC:ai Also known as: regulation of stress fibre formation, regulation of stress fibre biosynthesis